{
  "gene": "UniProtKB:Q96QF0",
  "term_id": "UNKNOWN:0002",
  "gene_name": "Rab-3A-interacting protein",
  "gene_symbol": "RAB3IP",
  "term_label": "Unknown biological process"
}